{
  "term_label": "transcription corepressor activity",
  "term_id": "GO:0003714",
  "gene": "UniProtKB:Q8N895",
  "gene_symbol": "ZNF366",
  "gene_name": "Zinc finger protein 366"
}